histamine receptor activity [GO:0004969] (MF) Sources: GOC:ai Definition: Combining with histamine to initiate a change in cell activity. Histamine is a physiologically active amine, found in plant and animal tissue and released from mast cells as part of an allergic reaction in humans. Relationships: is a type of GO:0008227; has part histamine binding [GO:0051381]